{
  "gene_symbol": "PCDHGA11",
  "gene_name": "Protocadherin gamma-A11",
  "gene": "UniProtKB:Q9Y5H2",
  "term_label": "plasma membrane",
  "term_id": "GO:0005886"
}